principal sensory nucleus of trigeminal nerve development [GO:0021740] (biological process) Note: Note that this term was placed as a child of 'brain development' because the nucleus spans multiple brain regions. Also known as: pontine nucleus development Sources: GOC:cls, GOC:curators, GOC:dgh, GOC:dph, GOC:jid Definition: The process whose specific outcome is the progression of the pontine nucleus over time, from its formation to the mature structure. Relationships: is_a trigeminal sensory nucleus development [GO:0021730]